{
  "term_label": "Unknown molecular function",
  "gene_symbol": "PPFIA4",
  "gene": "UniProtKB:O75335",
  "term_id": "UNKNOWN:0001",
  "gene_name": "Liprin-alpha-4"
}